phosphatidylethanolamine lysophospholipase activity [GO:0120559] (molecular function) Definition: Catalysis of the reaction: a 1-acyl-sn-glycero-3-phosphoethanolamine + H2O = sn-glycero-3-phosphoethanolamine + a fatty acid + H+. Sources: RHEA:32967 Relationships: is a type of GO:0120558